negative regulation of cGAS/STING signaling pathway [GO:0160049] (biological process) References: PMID:29875158 Relationships: is a type of negative regulation of cytoplasmic pattern recognition receptor signaling pathway [GO:0039532]; RO_0002212 cGAS/STING signaling pathway [GO:0140896] Definition: Any process that stops, prevents or reduces the frequency, rate or extent of cGAS/STING signaling pathway.